{
  "gene_symbol": "ATP8A2",
  "gene": "UniProtKB:Q9NTI2",
  "gene_name": "Phospholipid-transporting ATPase IB",
  "term_id": "GO:0140326",
  "term_label": "ATPase-coupled intramembrane lipid transporter activity"
}